{
  "gene_name": "6-phosphofructo-2-kinase_fructose-2,6-bisphosphatase 4",
  "gene": "UniProtKB:Q16877",
  "term_label": "fructose 2,6-bisphosphate metabolic process",
  "gene_symbol": "PFKFB4",
  "term_id": "GO:0006003"
}